{
  "term_id": "GO:0006974",
  "gene_name": "Fanconi anemia group G protein",
  "gene": "UniProtKB:O15287",
  "term_label": "DNA damage response",
  "gene_symbol": "FANCG"
}